{
  "term_id": "GO:0031261",
  "gene_name": "Origin recognition complex subunit 3",
  "gene_symbol": "ORC3",
  "term_label": "DNA replication preinitiation complex",
  "gene": "UniProtKB:Q9UBD5"
}